{
  "gene_symbol": "CLPTM1L",
  "gene_name": "Lipid scramblase CLPTM1L",
  "term_label": "endomembrane system",
  "term_id": "GO:0012505",
  "gene": "UniProtKB:Q96KA5"
}